{
  "gene_name": "Serine_threonine-protein kinase RIO1",
  "gene": "UniProtKB:Q9BRS2",
  "gene_symbol": "RIOK1",
  "term_label": "cytosol",
  "term_id": "GO:0005829"
}